{
  "term_label": "phosphoric diester hydrolase activity",
  "gene": "UniProtKB:P27695",
  "gene_name": "DNA-(apurinic or apyrimidinic site) endonuclease",
  "term_id": "GO:0008081",
  "gene_symbol": "APEX1"
}